eukaryotic translation initiation factor 3 complex, eIF3e [GO:0071540] (cellular component) References: PMID:15904532, PMID:19061185 Relationships: is_a eukaryotic translation initiation factor 3 complex [GO:0005852] Also known as: eIF3e-containing eukaryotic translation initiation factor 3 complex Definition: An eukaryotic translation initiation factor 3 complex that contains the PCI-domain protein eIF3e.